{
  "gene_name": "Carbohydrate-responsive element-binding protein",
  "gene_symbol": "MLXIPL",
  "gene": "UniProtKB:Q9NP71",
  "term_id": "GO:0000981",
  "term_label": "DNA-binding transcription factor activity, RNA polymerase II-specific"
}